{
  "gene_name": "Coiled-coil domain-containing protein 7",
  "term_id": "UNKNOWN:0003",
  "gene_symbol": "CCDC7",
  "gene": "UniProtKB:Q96M83",
  "term_label": "Unknown cellular component"
}